{
  "gene": "UniProtKB:P41226",
  "gene_name": "Ubiquitin-like modifier-activating enzyme 7",
  "gene_symbol": "UBA7",
  "term_id": "GO:0045087",
  "term_label": "innate immune response"
}